{
  "term_label": "nucleus",
  "term_id": "GO:0005634",
  "gene_name": "PHD finger protein 3",
  "gene": "UniProtKB:Q92576",
  "gene_symbol": "PHF3"
}